{
  "gene_symbol": "GAS2L1",
  "gene": "UniProtKB:Q99501",
  "gene_name": "GAS2-like protein 1",
  "term_label": "microtubule plus-end",
  "term_id": "GO:0035371"
}